{
  "gene": "UniProtKB:O60602",
  "term_label": "toll-like receptor signaling pathway",
  "term_id": "GO:0002224",
  "gene_name": "Toll-like receptor 5",
  "gene_symbol": "TLR5"
}